transmembrane receptor protein phosphatase activity [GO:0019198] (molecular function) Sources: GOC:hjd Subtypes: GO:0005001 Relationships: is a type of GO:0004721; is_a transmembrane signaling receptor activity [GO:0004888] Definition: Combining with a signal and transmitting the signal from one side of the membrane to the other to initiate a change in cell activity by catalysis of the reaction: a phosphoprotein + H2O = a protein + phosphate.